lateral pseudopodium retraction [GO:0120320] (biological process) Also known as: lateral pseudopodium suppression Relationships: is a type of GO:0031270 Definition: The myosin-based contraction and retraction of a lateral pseudopodium. References: PMID:12953059, PMID:15483055, PMID:17623773 Sources: GOC:krc, GOC:pf